{
  "gene_name": "Complement C1q-like protein 3",
  "term_id": "UNKNOWN:0001",
  "gene_symbol": "C1QL3",
  "term_label": "Unknown molecular function",
  "gene": "UniProtKB:Q5VWW1"
}